{
  "gene_symbol": "PDZRN4",
  "gene_name": "PDZ domain-containing RING finger protein 4",
  "term_label": "Unknown cellular component",
  "gene": "UniProtKB:Q6ZMN7",
  "term_id": "UNKNOWN:0003"
}